{
  "gene_symbol": "SLC7A5P2",
  "gene_name": "Putative L-type amino acid transporter 1-like protein IMAA",
  "term_label": "Unknown cellular component",
  "term_id": "UNKNOWN:0003",
  "gene": "UniProtKB:Q9GIP4"
}